{
  "gene": "UniProtKB:O75717",
  "term_id": "GO:0000278",
  "gene_name": "WD repeat and HMG-box DNA-binding protein 1",
  "gene_symbol": "WDHD1",
  "term_label": "mitotic cell cycle"
}